positive regulation of clathrin-dependent endocytosis [GO:2000370] (biological process) Sources: GOC:BHF, GOC:mah Also known as: positive regulation of clathrin coated pit-dependent endocytosis, positive regulation of clathrin-mediated endocytosis Relationships: is_a positive regulation of receptor-mediated endocytosis [GO:0048260]; is a type of regulation of clathrin-dependent endocytosis [GO:2000369]; positively regulates clathrin-dependent endocytosis [GO:0072583] Definition: Any process that activates or increases the frequency, rate or extent of clathrin-mediated endocytosis.